membrane repolarization [GO:0086009] (biological process) Sources: GOC:BHF, GOC:mtg_cardiac_conduct_nov11 Definition: The process in which ions are transported across a membrane such that the membrane potential changes in the repolarizing direction, toward the steady state potential. For example, the repolarization during an action potential is from a positive membrane potential towards a negative resting potential. Subtypes: GO:0086011, cardiac muscle cell membrane repolarization [GO:0099622] Relationships: is a type of GO:0042391 Regulation: regulated by regulation of membrane repolarization [GO:0060306]